{
  "term_label": "plasma membrane",
  "gene_symbol": "PACSIN1",
  "term_id": "GO:0005886",
  "gene": "UniProtKB:Q9BY11",
  "gene_name": "Protein kinase C and casein kinase substrate in neurons protein 1"
}